{
  "gene": "UniProtKB:Q96NA8",
  "term_id": "GO:0008021",
  "gene_name": "t-SNARE domain-containing protein 1",
  "gene_symbol": "TSNARE1",
  "term_label": "synaptic vesicle"
}